{
  "gene": "UniProtKB:P16150",
  "term_label": "Unknown molecular function",
  "gene_symbol": "SPN",
  "term_id": "UNKNOWN:0001",
  "gene_name": "Leukosialin"
}